negative regulation of endosome organization [GO:1904979] (biological process) References: PMID:22511594 Sources: GOC:PARL, GOC:TermGenie, GOC:pad, GO_REF:0000058 Relationships: is a type of negative regulation of organelle organization [GO:0010639]; is a type of regulation of endosome organization [GO:1904978]; negatively regulates endosome organization [GO:0007032] Definition: Any process that stops, prevents or reduces the frequency, rate or extent of endosome organization. Subtypes: GO:1905366 Also known as: down regulation of endosome organisation, down regulation of endosome organization, down-regulation of endosome organisation, down-regulation of endosome organization, downregulation of endosome organisation, downregulation of endosome organization, negative regulation of endosome organisation, inhibition of endosome organisation, inhibition of endosome organization, down regulation of endosome organization and biogenesis, down-regulation of endosome organization and biogenesis, downregulation of endosome organization and biogenesis, inhibition of endosome organization and biogenesis, negative regulation of endosome organization and biogenesis